{
  "gene": "UniProtKB:Q8IWB7",
  "gene_symbol": "WDFY1",
  "term_id": "UNKNOWN:0001",
  "term_label": "Unknown molecular function",
  "gene_name": "WD repeat and FYVE domain-containing protein 1"
}